{
  "term_id": "GO:0006364",
  "gene_name": "Probable ATP-dependent RNA helicase DDX47",
  "gene": "UniProtKB:Q9H0S4",
  "term_label": "rRNA processing",
  "gene_symbol": "DDX47"
}